{
  "term_label": "Unknown cellular component",
  "gene_symbol": "PLGLA",
  "term_id": "UNKNOWN:0003",
  "gene": "UniProtKB:Q15195",
  "gene_name": "Plasminogen-like protein A"
}